{
  "term_id": "GO:0071320",
  "term_label": "cellular response to cAMP",
  "gene_symbol": "CRTC2",
  "gene": "UniProtKB:Q53ET0",
  "gene_name": "CREB-regulated transcription coactivator 2"
}